ATP-dependent diacylglycerol kinase activity [GO:0004143] (molecular function) Definition: Catalysis of the reaction: a 1,2-diacyl-sn-glycerol + ATP = a 1,2-diacyl-sn-glycero-3-phosphate + ADP + H+. Sources: GOC:elh, RHEA:10272 Also known as: diacylglycerol kinase activity, diglyceride kinase activity, diacylglycerol kinase activity (ATP), DGK activity Relationships: is a type of GO:0001727; is_a phosphotransferase activity, alcohol group as acceptor [GO:0016773]